{
  "gene": "UniProtKB:P24071",
  "gene_name": "Immunoglobulin alpha Fc receptor",
  "gene_symbol": "FCAR",
  "term_id": "GO:0005886",
  "term_label": "plasma membrane"
}